{
  "gene": "UniProtKB:O14924",
  "term_label": "nucleus",
  "term_id": "GO:0005634",
  "gene_name": "Regulator of G-protein signaling 12",
  "gene_symbol": "RGS12"
}